{
  "gene": "UniProtKB:Q99999",
  "term_label": "myelination",
  "gene_name": "Galactosylceramide sulfotransferase",
  "gene_symbol": "GAL3ST1",
  "term_id": "GO:0042552"
}